{
  "gene": "UniProtKB:O75342",
  "term_label": "arachidonate 12(S)-lipoxygenase activity",
  "gene_symbol": "ALOX12B",
  "gene_name": "Arachidonate 12-lipoxygenase, 12R-type",
  "term_id": "GO:0004052"
}